phosphocholine hydrolase activity [GO:0044606] (molecular function) Definition: Catalysis of the reaction: protein-serine-choline phosphate + H2O = protein-serine + choline phosphate. References: PMID:22158903 Sources: GOC:sp Relationships: is a type of hydrolase activity, acting on acid anhydrides, in phosphorus-containing anhydrides [GO:0016818]